regulation of interleukin-22 production [GO:0032666] (biological process) Also known as: regulation of IL-22 production, regulation of interleukin-22 biosynthetic process Sources: GOC:mah Subtypes: negative regulation of interleukin-22 production [GO:0032706], GO:0032746 Relationships: is_a regulation of cytokine production [GO:0001817]; regulates GO:0032626 Definition: Any process that modulates the frequency, rate, or extent of interleukin-22 production.